{
  "gene": "UniProtKB:Q9GZY8",
  "term_label": "Unknown molecular function",
  "term_id": "UNKNOWN:0001",
  "gene_symbol": "MFF",
  "gene_name": "Mitochondrial fission factor"
}